{
  "term_id": "GO:0030509",
  "term_label": "BMP signaling pathway",
  "gene": "UniProtKB:Q15797",
  "gene_symbol": "SMAD1",
  "gene_name": "Mothers against decapentaplegic homolog 1"
}